{
  "gene_name": "Endoplasmic reticulum-Golgi intermediate compartment protein 1",
  "term_label": "COPII-coated ER to Golgi transport vesicle",
  "gene": "UniProtKB:Q969X5",
  "gene_symbol": "ERGIC1",
  "term_id": "GO:0030134"
}